{
  "gene_symbol": "EXOC3L1",
  "gene_name": "Exocyst complex component 3-like protein",
  "gene": "UniProtKB:Q86VI1",
  "term_id": "GO:0000145",
  "term_label": "exocyst"
}